{
  "term_label": "cholesterol binding",
  "term_id": "GO:0015485",
  "gene_name": "StAR-related lipid transfer protein 3",
  "gene": "UniProtKB:Q14849",
  "gene_symbol": "STARD3"
}